SOD1-Bcl-2 complex [GO:0033607] (cellular component) References: PMID:15233914, PMID:16790527 Definition: A heterodimeric protein complex formed of superoxide dismutase 1 and Bcl-2. Complex formation is thought to link superoxide dismutase to an apoptotic pathway. Relationships: is a type of intracellular protein-containing complex [GO:0140535]